{
  "term_label": "structural constituent of myelin sheath",
  "gene_symbol": "MALL",
  "gene_name": "MAL-like protein",
  "term_id": "GO:0019911",
  "gene": "UniProtKB:Q13021"
}